{
  "gene_symbol": "DDB2",
  "term_id": "GO:0003684",
  "term_label": "damaged DNA binding",
  "gene_name": "DNA damage-binding protein 2",
  "gene": "UniProtKB:Q92466"
}